cytoplasmic microtubule plus-end [GO:1904511] (cellular component) References: PMID:15772152 Sources: GOC:TermGenie, GO_REF:0000064 Relationships: is a type of microtubule plus-end [GO:0035371]; is part of cytoplasmic microtubule [GO:0005881] Definition: Any microtubule plus-end that is part of a cytoplasmic microtubule. Subtypes: cortical microtubule plus-end [GO:1903754] Also known as: growing microtubule plus end of cytoplasmic microtubule, microtubule plus end of cytoplasmic microtubule, microtubule plus-end of cytoplasmic microtubule, growing microtubule plus end of non-spindle-associated astral microtubule, microtubule plus end of non-spindle-associated astral microtubule, microtubule plus-end of non-spindle-associated astral microtubule